sn-glycerol-3-phosphate 2-alpha-galactosyltransferase activity [GO:0047221] (molecular function) Definition: Catalysis of the reaction: sn-glycerol 3-phosphate + UDP-D-galactose = 2-(alpha-D-galactosyl)-sn-glycerol 3-phosphate + H+ + UDP. Relationships: is a type of UDP-galactosyltransferase activity [GO:0035250] Sources: EC:2.4.1.137, RHEA:14285 Also known as: FPS, UDP-galactose, sn-3-glycerol phosphate:1->2' galactosyltransferase activity, UDP-galactose:sn-glycerol-3-phosphate 2-alpha-D-galactosyltransferase activity, UDP-galactose:sn-glycerol-3-phosphate-2-D-galactosyl transferase activity, UDPgalactose:sn-glycerol-3-phosphate 2-alpha-D-galactosyltransferase activity, floridoside phosphate synthase activity, floridoside phosphate synthetase activity, floridoside-phosphate synthase activity